{
  "term_label": "RNA polymerase II cis-regulatory region sequence-specific DNA binding",
  "gene": "UniProtKB:Q96G25",
  "gene_symbol": "MED8",
  "gene_name": "Mediator of RNA polymerase II transcription subunit 8",
  "term_id": "GO:0000978"
}